galactose biosynthetic process [GO:0046369] (BP) Definition: The chemical reactions and pathways resulting in the formation of galactose, the aldohexose galacto-hexose. Subtypes: beta-D-galactofuranose biosynthetic process [GO:1901358] Sources: ISBN:0198506732 Also known as: galactose anabolism, galactose biosynthesis, galactose formation, galactose synthesis Relationships: is a type of galactose metabolic process [GO:0006012]; is a type of hexose biosynthetic process [GO:0019319]